canalicular bile acid transmembrane transporter activity [GO:0015126] (molecular function) Sources: GOC:dph Definition: The directed movement of bile acid and bile salts out of a hepatocyte and into the bile canaliculus by means of an agent such as a transporter or pore. Bile canaliculi are the thin tubes formed by hepatocyte membranes. Bile acids are any of a group of steroid carboxylic acids occurring in bile, where they are present as the sodium salts of their amides with glycine or taurine. Relationships: is_a bile acid transmembrane transporter activity [GO:0015125]; is part of canalicular bile acid transport [GO:0015722]